{
  "term_id": "GO:0002244",
  "term_label": "hematopoietic progenitor cell differentiation",
  "gene_symbol": "PRRC2C",
  "gene": "UniProtKB:Q9Y520",
  "gene_name": "Protein PRRC2C"
}